{
  "term_id": "GO:0005737",
  "gene": "UniProtKB:Q8N987",
  "gene_name": "N-terminal EF-hand calcium-binding protein 1",
  "gene_symbol": "NECAB1",
  "term_label": "cytoplasm"
}